positive regulation of norepinephrine secretion [GO:0010701] (biological process) Relationships: is a type of regulation of norepinephrine secretion [GO:0014061]; is a type of GO:0033605; RO_0002213 norepinephrine secretion [GO:0048243] Sources: GOC:dph, GOC:tb Definition: Any process that increases the frequency, rate or extent of the regulated release of norepinephrine.